{
  "term_id": "GO:0008076",
  "gene_symbol": "KCNV1",
  "gene": "UniProtKB:Q6PIU1",
  "gene_name": "Potassium voltage-gated channel subfamily V member 1",
  "term_label": "voltage-gated potassium channel complex"
}